{
  "term_id": "GO:0060337",
  "term_label": "type I interferon-mediated signaling pathway",
  "gene_symbol": "OAS1",
  "gene_name": "2'-5'-oligoadenylate synthase 1",
  "gene": "UniProtKB:P00973"
}